cellular response to prolactin [GO:1990646] (biological process) Definition: Any process that results in a change in state or activity of a cell (in terms of movement, secretion, enzyme production, gene expression, etc.) as a result of a prolactin stimulus. References: PMID:7760850 Relationships: is a type of cellular response to peptide hormone stimulus [GO:0071375]; is a type of response to prolactin [GO:1990637]